posterior abdomen determination [GO:0007359] (BP) Definition: The regionalization process in which the posterior (abdominal) regions of the embryo are specified by the gap genes. Relationships: is a type of GO:0009952; is part of GO:0007354 Sources: GOC:dph, GOC:isa_complete, ISBN:0879694238, http://fly.ebi.ac.uk/allied-data/lk/interactive-fly/aimain/1aahome.htm Note: Note that this process is exemplified in insects by the actions of the knirps gene product.